{
  "gene_symbol": "AGAP3",
  "term_id": "GO:0043161",
  "gene_name": "Arf-GAP with GTPase, ANK repeat and PH domain-containing protein 3",
  "term_label": "proteasome-mediated ubiquitin-dependent protein catabolic process",
  "gene": "UniProtKB:Q96P47"
}